{
  "gene": "UniProtKB:P06241",
  "gene_symbol": "FYN",
  "gene_name": "Tyrosine-protein kinase Fyn",
  "term_id": "GO:0050852",
  "term_label": "T cell receptor signaling pathway"
}